{
  "term_label": "DNA-binding transcription factor activity, RNA polymerase II-specific",
  "gene_name": "Zinc finger protein GLI4",
  "term_id": "GO:0000981",
  "gene_symbol": "GLI4",
  "gene": "UniProtKB:P10075"
}